{
  "gene_symbol": "NKRF",
  "gene_name": "NF-kappa-B-repressing factor",
  "term_label": "negative regulation of DNA-templated transcription",
  "term_id": "GO:0045892",
  "gene": "UniProtKB:O15226"
}